triglyceride catabolic process [GO:0019433] (biological process) Relationships: is a type of triglyceride metabolic process [GO:0006641]; is a type of acylglycerol catabolic process [GO:0046464] Sources: ISBN:0198506732 Definition: The chemical reactions and pathways resulting in the breakdown of a triglyceride, any triester of glycerol. Regulation: regulated by regulation of triglyceride catabolic process [GO:0010896]; negatively regulated by negative regulation of triglyceride catabolic process [GO:0010897]; positively regulated by positive regulation of triglyceride catabolic process [GO:0010898] Also known as: triacylglycerol catabolic process, triacylglycerol catabolism, triglyceride breakdown, triglyceride catabolism, triglyceride degradation